{
  "gene_name": "CSC1-like protein 2",
  "gene_symbol": "TMEM63B",
  "term_label": "Unknown biological process",
  "gene": "UniProtKB:Q5T3F8",
  "term_id": "UNKNOWN:0002"
}